phosphatidylethanolamine biosynthetic process [GO:0006646] (BP) Subtypes: phosphatidyl-N-monomethylethanolamine biosynthetic process [GO:0006647], dihydrosphingosine-1-P pathway [GO:0006648] Definition: The chemical reactions and pathways resulting in the formation of phosphatidylethanolamine, any of a class of glycerophospholipids in which a phosphatidyl group is esterified to the hydroxyl group of ethanolamine. Also known as: phosphatidylethanolamine anabolism, phosphatidylethanolamine biosynthesis, phosphatidylethanolamine formation, phosphatidylethanolamine synthesis Sources: ISBN:0198506732 Relationships: is a type of GO:0046337; is a type of glycerophospholipid biosynthetic process [GO:0046474]